{
  "term_id": "GO:0005102",
  "gene_symbol": "NXPH3",
  "term_label": "signaling receptor binding",
  "gene_name": "Neurexophilin-3",
  "gene": "UniProtKB:O95157"
}